intestinal stem cell homeostasis [GO:0036335] (biological process) Definition: Any biological process involved in the maintenance of the steady-state number of intestinal stem cells within a population of cells. References: PMID:22042863, PMID:22608824 Sources: GOC:nhn Also known as: intestinal crypt stem cell homeostasis Relationships: is a type of GO:0048872